{
  "gene_name": "YY1-associated protein 1",
  "gene_symbol": "YY1AP1",
  "term_id": "UNKNOWN:0003",
  "term_label": "Unknown cellular component",
  "gene": "UniProtKB:Q9H869"
}